{
  "gene_name": "Motor neuron and pancreas homeobox protein 1",
  "gene": "UniProtKB:P50219",
  "term_label": "endocrine pancreas development",
  "gene_symbol": "MNX1",
  "term_id": "GO:0031018"
}